{
  "gene_symbol": "SLC12A3",
  "gene_name": "Solute carrier family 12 member 3",
  "term_id": "GO:0006884",
  "term_label": "cell volume homeostasis",
  "gene": "UniProtKB:P55017"
}